{
  "term_label": "Unknown cellular component",
  "term_id": "UNKNOWN:0003",
  "gene_symbol": "EXTL2",
  "gene_name": "Exostosin-like 2",
  "gene": "UniProtKB:Q9UBQ6"
}